antigen processing and presentation via MHC class Ib [GO:0002475] (biological process) Subtypes: antigen processing and presentation of peptide antigen via MHC class Ib [GO:0002428], antigen processing and presentation of lipid antigen via MHC class Ib [GO:0048003] Definition: The process in which an antigen-presenting cell expresses antigen (peptide or lipid) on its cell surface in association with an MHC class Ib protein complex. Class Ib here refers to non-classical class I molecules, such as those of the CD1 or HLA-E gene families. Regulation: regulated by regulation of antigen processing and presentation via MHC class Ib [GO:0002592]; RO_0002212 by negative regulation of antigen processing and presentation via MHC class Ib [GO:0002593]; positively regulated by positive regulation of antigen processing and presentation via MHC class Ib [GO:0002594] References: PMID:15928678, PMID:15928680 Sources: GOC:add Relationships: is a type of antigen processing and presentation [GO:0019882]